{
  "gene_symbol": "IQCC",
  "term_id": "UNKNOWN:0002",
  "gene_name": "IQ domain-containing protein C",
  "gene": "UniProtKB:Q4KMZ1",
  "term_label": "Unknown biological process"
}